{
  "gene": "UniProtKB:P01350",
  "term_label": "G protein-coupled receptor signaling pathway",
  "term_id": "GO:0007186",
  "gene_name": "Gastrin",
  "gene_symbol": "GAST"
}